2-deoxyribose 1-phosphate biosynthetic process [GO:0006016] (biological process) Definition: The chemical reactions and pathways resulting in the formation of 2-deoxyribose 1-phosphate, the phosphorylated sugar 1-phospho-2-deoxyribose. Relationships: is a type of GO:0046385 Sources: ISBN:0198506732 Also known as: 2-deoxyribose 1-phosphate anabolism, 2-deoxyribose 1-phosphate biosynthesis, 2-deoxyribose 1-phosphate formation, 2-deoxyribose 1-phosphate synthesis